{
  "gene": "UniProtKB:P37088",
  "term_label": "ligand-gated sodium channel activity",
  "term_id": "GO:0015280",
  "gene_name": "Amiloride-sensitive sodium channel subunit alpha",
  "gene_symbol": "SCNN1A"
}